antisense RNA transcript catabolic process [GO:0071041] (biological process) Definition: The chemical reactions and pathways resulting in the breakdown of antisense transcripts, i.e. transcripts that were produced from the antisense strand of a gene that produces a gene product and which often have a regulatory effect on the transcription of that gene product. Sources: GOC:dgf, GOC:krc Relationships: is a type of antisense RNA metabolic process [GO:0042868]; is a type of nuclear RNA surveillance [GO:0071027] Subtypes: nuclear polyadenylation-dependent antisense transcript catabolic process [GO:0071040]